{
  "gene": "UniProtKB:Q9BZK7",
  "gene_name": "F-box-like_WD repeat-containing protein TBL1XR1",
  "term_id": "GO:0006357",
  "gene_symbol": "TBL1XR1",
  "term_label": "regulation of transcription by RNA polymerase II"
}